{
  "term_id": "GO:0000727",
  "term_label": "double-strand break repair via break-induced replication",
  "gene": "UniProtKB:Q14566",
  "gene_symbol": "MCM6",
  "gene_name": "DNA replication licensing factor MCM6"
}